plasma membrane bounded cell projection [GO:0120025] (cellular component) Sources: GOC:krc Definition: A prolongation or process extending from a cell and that is bounded by plasma membrane, e.g. a cilium, lamellipodium, or axon. Subtypes: ruffle [GO:0001726], uropod [GO:0001931], cilium [GO:0005929], mating projection [GO:0005937], rhabdomere [GO:0016028], lamellipodium [GO:0030027], pseudopodium [GO:0031143], bleb [GO:0032059], cytoneme [GO:0035230], root hair [GO:0035618], muscle cell projection [GO:0036194], neuron projection [GO:0043005], GO:0044393, cell hair [GO:0070451], macropinocytic cup [GO:0070685], GO:0090406, glial cell projection [GO:0097386], dendritic cell dendrite [GO:0097511], podocyte foot [GO:0098846], GO:0098854, actin-based cell projection [GO:0098858], GO:0120327, dinoflagellate peduncle [GO:1990905] Relationships: is a type of GO:0042995; has part plasma membrane region [GO:0098590]